{
  "term_id": "UNKNOWN:0003",
  "gene": "UniProtKB:O75828",
  "term_label": "Unknown cellular component",
  "gene_symbol": "CBR3",
  "gene_name": "Carbonyl reductase [NADPH] 3"
}